{
  "term_label": "protein maturation",
  "gene": "UniProtKB:Q9BRT8",
  "term_id": "GO:0051604",
  "gene_symbol": "ZNG1A",
  "gene_name": "Zinc-regulated GTPase metalloprotein activator 1A"
}